ligand-independent adenylate cyclase-activating G protein-coupled receptor signaling pathway [GO:0038035] (biological process) References: PMID:12402500, PMID:17629961 Relationships: is a type of GO:0007189; is a type of signal transduction in absence of ligand [GO:0038034] Also known as: G protein-coupled receptor signaling in absence of ligand, G-protein coupled receptor signaling in absence of agonist, G-protein coupled receptor signaling in absence of ligand, G-protein coupled receptor signalling in absence of ligand, basal G-protein coupled receptor signaling Definition: A G protein-coupled receptor signaling pathway in which the receptor constitutively activates adenylate cyclase, without binding to an agonist.